{
  "gene_name": "Protein disulfide-isomerase TMX3",
  "gene_symbol": "TMX3",
  "gene": "UniProtKB:Q96JJ7",
  "term_label": "endoplasmic reticulum",
  "term_id": "GO:0005783"
}